zygospore formation [GO:0034296] (BP) References: PMID:21858438 Sources: GOC:ds, GOC:mah Definition: The process in which zygospores are formed. Zygospores are characteristic of the zygomycete fungi (phylum Zygomycota) thick-walled and darkly colored, and usually heavily ornamented as well, with many spines or ridges. It is formed between two specialized organs called suspensors, which are themselves usually heavily ornamented, one from each mating partner. The zygospore forms between them and then breaks away. Relationships: is a type of GO:0043935 Regulation: regulated by regulation of zygospore formation [GO:0075298]; positively regulated by GO:0075299; negatively regulated by negative regulation of zygospore formation [GO:0075300]